{
  "gene_name": "Two pore channel protein 2",
  "term_label": "intracellularly phosphatidylinositol-3,5-bisphosphate-gated monatomic cation channel activity",
  "term_id": "GO:0097682",
  "gene_symbol": "TPCN2",
  "gene": "UniProtKB:Q8NHX9"
}